pyroglutamyl-peptidase activity [GO:0016920] (molecular function) Relationships: is a type of cysteine-type peptidase activity [GO:0008234]; is_a omega peptidase activity [GO:0008242] References: PMID:9920379 Sources: GOC:mah Definition: Catalysis of the release of the N-terminal pyroglutamyl group from a peptide or protein.